{
  "gene_name": "Vesicular, overexpressed in cancer, prosurvival protein 1",
  "term_id": "UNKNOWN:0001",
  "term_label": "Unknown molecular function",
  "gene": "UniProtKB:Q96AW1",
  "gene_symbol": "VOPP1"
}